{
  "term_id": "GO:0005634",
  "gene_symbol": "TEX15",
  "term_label": "nucleus",
  "gene": "UniProtKB:Q9BXT5",
  "gene_name": "Testis-expressed protein 15"
}